entrainment of circadian clock by photoperiod [GO:0043153] (biological process) Sources: GOC:jl Relationships: is_a photoperiodism [GO:0009648]; is a type of entrainment of circadian clock [GO:0009649] Definition: The synchronization of a circadian rhythm to photoperiod, the intermittent cycle of light (day) and dark (night). Also known as: photoentrainment of circadian clock